{
  "term_id": "GO:0019814",
  "gene_name": "Immunoglobulin kappa variable 2-30",
  "gene": "UniProtKB:P06310",
  "term_label": "immunoglobulin complex",
  "gene_symbol": "IGKV2-30"
}